{
  "gene_name": "Oxidative stress-responsive serine-rich protein 1",
  "term_id": "UNKNOWN:0003",
  "gene_symbol": "OSER1",
  "term_label": "Unknown cellular component",
  "gene": "UniProtKB:Q9NX31"
}